{
  "gene": "UniProtKB:O15354",
  "gene_name": "Prosaposin receptor GPR37",
  "term_id": "GO:0043235",
  "gene_symbol": "GPR37",
  "term_label": "receptor complex"
}